{
  "gene": "UniProtKB:Q8NHY3",
  "term_id": "GO:1904825",
  "gene_symbol": "GAS2L2",
  "term_label": "protein localization to microtubule plus-end",
  "gene_name": "GAS2-like protein 2"
}